response to low humidity [GO:0090547] (biological process) Relationships: is a type of response to humidity [GO:0009270] Definition: Any process that results in a change in state or activity of a cell or an organism (in terms of movement, secretion, enzyme production, gene expression, etc.) as a result of low humidity stimulus, reduced moisture in the atmosphere. Sources: GOC:tb